{
  "term_label": "negative regulation of phosphatidylinositol 3-kinase/protein kinase B signal transduction",
  "gene": "UniProtKB:Q9Y5J5",
  "gene_symbol": "PHLDA3",
  "term_id": "GO:0051898",
  "gene_name": "Pleckstrin homology-like domain family A member 3"
}